all-trans-phytoene synthase activity [GO:0140630] (molecular function) Relationships: is a type of pyrophosphatase activity [GO:0016462]; is part of carotenoid biosynthetic process [GO:0016117] References: PMID:12641468, PMID:7896759 Definition: Catalysis of the reaction: 2 geranylgeranyl diphosphate = all-trans-phytoene + 2 diphosphate. Also known as: phytoene synthase activity